{
  "gene_symbol": "TRPM3",
  "term_id": "GO:0005262",
  "gene_name": "Transient receptor potential cation channel subfamily M member 3",
  "gene": "UniProtKB:Q9HCF6",
  "term_label": "calcium channel activity"
}